{
  "gene": "UniProtKB:Q9UKJ8",
  "gene_name": "Disintegrin and metalloproteinase domain-containing protein 21",
  "term_label": "male gonad development",
  "term_id": "GO:0008584",
  "gene_symbol": "ADAM21"
}